{
  "term_label": "articular cartilage development",
  "term_id": "GO:0061975",
  "gene_symbol": "OPTC",
  "gene": "UniProtKB:Q9UBM4",
  "gene_name": "Opticin"
}